{
  "gene": "UniProtKB:Q9H902",
  "term_id": "GO:0005789",
  "gene_name": "Receptor expression-enhancing protein 1",
  "term_label": "endoplasmic reticulum membrane",
  "gene_symbol": "REEP1"
}